{
  "gene_symbol": "CDK16",
  "gene": "UniProtKB:Q00536",
  "gene_name": "Cyclin-dependent kinase 16",
  "term_label": "regulation of cell cycle phase transition",
  "term_id": "GO:1901987"
}